{
  "term_id": "GO:0005243",
  "term_label": "gap junction channel activity",
  "gene_name": "Gap junction gamma-2 protein",
  "gene": "UniProtKB:Q5T442",
  "gene_symbol": "GJC2"
}